{
  "term_label": "protein localization to endosome",
  "gene_name": "ADP-ribosylation factor 6",
  "gene": "UniProtKB:P62330",
  "term_id": "GO:0036010",
  "gene_symbol": "ARF6"
}